{
  "gene_name": "Ornithine aminotransferase, mitochondrial",
  "gene_symbol": "OAT",
  "gene": "UniProtKB:P04181",
  "term_id": "GO:0019544",
  "term_label": "L-arginine catabolic process to L-glutamate"
}